{
  "term_label": "vesicle fusion",
  "term_id": "GO:0006906",
  "gene_symbol": "GOSR2",
  "gene_name": "Golgi SNAP receptor complex member 2",
  "gene": "UniProtKB:O14653"
}